{
  "term_label": "Unknown biological process",
  "term_id": "UNKNOWN:0002",
  "gene_name": "Uncharacterized protein C19orf85",
  "gene_symbol": "C19orf85",
  "gene": "UniProtKB:A0A1B0GUS0"
}